{
  "term_id": "GO:0005975",
  "gene_symbol": "AMY2B",
  "gene_name": "Alpha-amylase 2B",
  "term_label": "carbohydrate metabolic process",
  "gene": "UniProtKB:P19961"
}